{
  "term_label": "defense response to Gram-positive bacterium",
  "gene": "UniProtKB:P49913",
  "gene_symbol": "CAMP",
  "term_id": "GO:0050830",
  "gene_name": "Cathelicidin antimicrobial peptide"
}